{
  "term_id": "GO:0007507",
  "gene_symbol": "ACVRL1",
  "term_label": "heart development",
  "gene": "UniProtKB:P37023",
  "gene_name": "Serine_threonine-protein kinase receptor R3"
}